intracellular cysteine homeostasis [GO:0080145] (biological process) Definition: A homeostatic process involved in the maintenance of a steady state level of cysteine within a cell. Relationships: is a type of intracellular amino acid homeostasis [GO:0080144] Also known as: cellular cysteine homeostasis, cysteine homeostasis References: PMID:19955263